{
  "gene_symbol": "OR4Q2",
  "gene_name": "Olfactory receptor 4Q2",
  "term_id": "GO:0004984",
  "term_label": "olfactory receptor activity",
  "gene": "UniProtKB:P0C623"
}